{
  "term_label": "negative regulation of transcription by RNA polymerase II",
  "gene_symbol": "ZBTB32",
  "term_id": "GO:0000122",
  "gene_name": "Zinc finger and BTB domain-containing protein 32",
  "gene": "UniProtKB:Q9Y2Y4"
}